{
  "gene_name": "Hydroperoxide isomerase ALOXE3",
  "term_id": "GO:0019372",
  "gene": "UniProtKB:Q9BYJ1",
  "gene_symbol": "ALOXE3",
  "term_label": "lipoxygenase pathway"
}